{
  "gene": "UniProtKB:Q8TF08",
  "gene_name": "Cytochrome c oxidase subunit 7B2, mitochondrial",
  "term_id": "UNKNOWN:0001",
  "gene_symbol": "COX7B2",
  "term_label": "Unknown molecular function"
}